{
  "term_id": "GO:0000977",
  "gene": "UniProtKB:Q15937",
  "term_label": "RNA polymerase II transcription regulatory region sequence-specific DNA binding",
  "gene_symbol": "ZNF79",
  "gene_name": "Zinc finger protein 79"
}